protein monoubiquitination [GO:0006513] (biological process) Definition: Addition of a single ubiquitin group to a protein. Also known as: protein monoubiquitinylation, protein monoubiquitylation Sources: GOC:ai Regulation: regulated by GO:1902525; negatively regulated by negative regulation of protein monoubiquitination [GO:1902526]; RO_0002213 by positive regulation of protein monoubiquitination [GO:1902527] Relationships: is a type of GO:0016567